{
  "gene_name": "Copper-transporting ATPase 2",
  "term_id": "GO:0043682",
  "gene": "UniProtKB:P35670",
  "gene_symbol": "ATP7B",
  "term_label": "P-type divalent copper transporter activity"
}